regulation of vulval development [GO:0040028] (BP) Relationships: is a type of regulation of developmental process [GO:0050793]; regulates GO:0040025 Definition: Any process that modulates the frequency, rate or extent of development of the vulva. Vulval development is the process whose specific outcome is the progression of the egg-laying organ of female and hermaphrodite nematodes over time, from its formation to the mature structure. In nematodes, the vulva is formed from ventral epidermal cells during larval stages to give rise to a fully formed vulva in the adult. Subtypes: positive regulation of vulval development [GO:0040026], GO:0040027 Sources: GOC:kmv, GOC:ma